taxoid 2alpha-hydroxylase activity [GO:0102365] (molecular function) Definition: Catalysis of the reaction: taxusin + NADPH + O2 + H+ = 2-alpha-hydroxytaxusin + NADP + H2O. Also converts 7beta-hydroxytaxusin to 2alpha,7beta-dihydroxytaxusin. References: PMID:15178487 Sources: EC:1.14.14.183 Relationships: is a type of oxidoreductase activity, acting on paired donors, with incorporation or reduction of molecular oxygen, reduced flavin or flavoprotein as one donor, and incorporation of one atom of oxygen [GO:0016712] Also known as: taxusin 2-alpha-hydroxylase activity